{
  "term_label": "muscle cell cellular homeostasis",
  "term_id": "GO:0046716",
  "gene": "UniProtKB:Q13496",
  "gene_name": "Myotubularin",
  "gene_symbol": "MTM1"
}